proteasome localization [GO:0031144] (biological process) Definition: Any process in which the proteasome is transported to, or maintained in, a specific location. Sources: GOC:mah Relationships: is a type of protein-containing complex localization [GO:0031503] Also known as: establishment and maintenance of proteasome localization, proteasome localisation